{
  "term_label": "RNA polymerase II transcription regulator complex",
  "gene_name": "Achaete-scute homolog 5",
  "gene": "UniProtKB:Q7RTU5",
  "gene_symbol": "ASCL5",
  "term_id": "GO:0090575"
}